{
  "gene_symbol": "FAIM2",
  "term_label": "endoplasmic reticulum",
  "gene_name": "Protein lifeguard 2",
  "term_id": "GO:0005783",
  "gene": "UniProtKB:Q9BWQ8"
}